{
  "gene_symbol": "HRH3",
  "gene": "UniProtKB:Q9Y5N1",
  "term_id": "GO:0007268",
  "gene_name": "Histamine H3 receptor",
  "term_label": "chemical synaptic transmission"
}